{
  "gene": "UniProtKB:A8MQB3",
  "gene_name": "Putative uncharacterized protein LINC02693",
  "term_id": "UNKNOWN:0003",
  "gene_symbol": "LINC02693",
  "term_label": "Unknown cellular component"
}